{
  "gene_symbol": "WNT6",
  "term_label": "canonical Wnt signaling pathway",
  "gene": "UniProtKB:Q9Y6F9",
  "gene_name": "Protein Wnt-6",
  "term_id": "GO:0060070"
}